dendritic cell differentiation [GO:0097028] (biological process) Definition: The process in which a precursor cell type acquires the specialized features of a dendritic cell. A dendritic cell is a leukocyte of dendritic lineage specialized in the uptake, processing, and transport of antigens to lymph nodes for the purpose of stimulating an immune response via T cell activation. Sources: CL:0000451, GOC:pr Note: Note that immunologists typically use the word 'maturation' to refer to dendritic cells undergoing the process that GO describes as 'cell differentiation'. Relationships: is a type of mononuclear cell differentiation [GO:1903131] Subtypes: GO:0002273, GO:0043011, GO:0097029 Regulation: regulated by regulation of dendritic cell differentiation [GO:2001198]; negatively regulated by negative regulation of dendritic cell differentiation [GO:2001199]; positively regulated by positive regulation of dendritic cell differentiation [GO:2001200]